{
  "gene_name": "Golgi apparatus membrane protein TVP23 homolog A",
  "gene": "UniProtKB:A6NH52",
  "gene_symbol": "TVP23A",
  "term_label": "protein secretion",
  "term_id": "GO:0009306"
}